{
  "gene_symbol": "ZBTB49",
  "gene_name": "Zinc finger and BTB domain-containing protein 49",
  "term_label": "RNA polymerase II cis-regulatory region sequence-specific DNA binding",
  "gene": "UniProtKB:Q6ZSB9",
  "term_id": "GO:0000978"
}